{
  "gene_name": "Vesicle transport protein SEC20",
  "term_label": "endoplasmic reticulum",
  "gene": "UniProtKB:Q12981",
  "term_id": "GO:0005783",
  "gene_symbol": "BNIP1"
}